{
  "gene_name": "Transmembrane emp24 domain-containing protein 1",
  "gene_symbol": "TMED1",
  "gene": "UniProtKB:Q13445",
  "term_id": "GO:0005793",
  "term_label": "endoplasmic reticulum-Golgi intermediate compartment"
}